{
  "gene_name": "Interferon-induced protein with tetratricopeptide repeats 3",
  "gene_symbol": "IFIT3",
  "term_id": "GO:0003723",
  "term_label": "RNA binding",
  "gene": "UniProtKB:O14879"
}